symbiont-mediated suppression of host neutrophil extracellular trap formation [GO:0141145] (biological process) Relationships: is a type of symbiont-mediated perturbation of host cellular process [GO:0044068]; is a type of GO:0052031 Also known as: symbiont-mediated suppression of host neutrophil extracellular traps formation, symbiont-mediated perturbation of host neutrophil extracellular trap formation References: PMID:30038902, PMID:34108482 Definition: A process in which a symbiont inhibits or disrupts the formation of neutrophil extracellular traps by the host cell. The host is defined as the larger of the organisms involved in a symbiotic interaction.